positive regulation of dendritic spine maintenance [GO:1902952] (biological process) Definition: Any process that activates or increases the frequency, rate or extent of dendritic spine maintenance. Relationships: is a type of positive regulation of cell projection organization [GO:0031346]; is a type of GO:1902950; positively regulates dendritic spine maintenance [GO:0097062] Also known as: up regulation of dendritic spine maintenance, up-regulation of dendritic spine maintenance, upregulation of dendritic spine maintenance, activation of dendritic spine maintenance References: PMID:24328732 Sources: GOC:TermGenie, GOC:sjp, GO_REF:0000058